{
  "term_id": "GO:0045454",
  "term_label": "cell redox homeostasis",
  "gene_symbol": "PRDX3",
  "gene": "UniProtKB:P30048",
  "gene_name": "Thioredoxin-dependent peroxide reductase, mitochondrial"
}